{
  "gene_symbol": "RBP2",
  "gene": "UniProtKB:P50120",
  "term_label": "nucleus",
  "term_id": "GO:0005634",
  "gene_name": "Retinol-binding protein 2"
}